{
  "term_id": "GO:0045335",
  "gene_symbol": "RAB7B",
  "gene": "UniProtKB:Q96AH8",
  "term_label": "phagocytic vesicle",
  "gene_name": "Ras-related protein Rab-7b"
}